{
  "gene_symbol": "WHAMMP3",
  "term_id": "UNKNOWN:0002",
  "term_label": "Unknown biological process",
  "gene_name": "Putative WASP homolog-associated protein with actin, membranes and microtubules-like protein 1",
  "gene": "UniProtKB:Q1A5X7"
}